{
  "term_label": "adenosine to inosine editing",
  "gene": "UniProtKB:Q9NS39",
  "term_id": "GO:0006382",
  "gene_symbol": "ADARB2",
  "gene_name": "Double-stranded RNA-specific editase B2"
}